{
  "term_id": "GO:0005615",
  "gene_name": "Inhibin beta B chain",
  "term_label": "extracellular space",
  "gene_symbol": "INHBB",
  "gene": "UniProtKB:P09529"
}